{
  "gene_symbol": "NOTCH2NLC",
  "term_id": "GO:0021987",
  "gene": "UniProtKB:P0DPK4",
  "gene_name": "Notch homolog 2 N-terminal-like protein C",
  "term_label": "cerebral cortex development"
}